molybdenum cofactor cytidylyltransferase activity [GO:0061602] (molecular function) Sources: RHEA:31335 Relationships: is a type of cytidylyltransferase activity [GO:0070567] Definition: Catalysis of the reaction: Mo-molybdopterin + CTP + H+ = Mo-molybdopterin cytosine dinucleotide + diphosphate.